peptidyl-phenylalanine modification [GO:0018207] (biological process) Sources: GOC:go_curators Relationships: is a type of peptidyl-amino acid modification [GO:0018193] Definition: The modification of peptidyl-phenylalanine. Subtypes: peptidyl-L-3-phenyllactic acid biosynthetic process from peptidyl-phenylalanine [GO:0018061]